{
  "gene_symbol": "ZFYVE28",
  "term_id": "GO:0042059",
  "gene_name": "Lateral signaling target protein 2 homolog",
  "term_label": "negative regulation of epidermal growth factor receptor signaling pathway",
  "gene": "UniProtKB:Q9HCC9"
}